{
  "gene_name": "Zinc finger protein 841",
  "gene_symbol": "ZNF841",
  "gene": "UniProtKB:Q6ZN19",
  "term_id": "GO:0000122",
  "term_label": "negative regulation of transcription by RNA polymerase II"
}